P granule organization [GO:0030719] (biological process) Definition: A process that is carried out at the cellular level which results in the assembly, arrangement of constituent parts, or disassembly of polar granules, cytoplasmic, non-membranous RNA/protein complex aggregates in the primordial germ cells of many higher eukaryotes. Also known as: polar granule organisation, polar granule organization and biogenesis, P granule organization and biogenesis Subtypes: P granule assembly [GO:1903863], P granule disassembly [GO:1903864] Relationships: is a type of GO:0006996; is part of pole plasm assembly [GO:0007315] References: PMID:10851135, PMID:770367